{
  "term_id": "GO:0005846",
  "gene_symbol": "NCBP2",
  "gene_name": "Nuclear cap-binding protein subunit 2",
  "term_label": "nuclear cap binding complex",
  "gene": "UniProtKB:P52298"
}